{
  "term_label": "Unknown cellular component",
  "gene_name": "Keratin-associated protein 3-3",
  "term_id": "UNKNOWN:0003",
  "gene_symbol": "KRTAP3-3",
  "gene": "UniProtKB:Q9BYR6"
}